tRNA-dihydrouridine16 synthase activity [GO:0102262] (MF) Relationships: is a type of tRNA dihydrouridine synthase activity [GO:0017150] Sources: GOC:pz Definition: Catalysis of the reaction: a 5,6-dihydrouracil16 in tRNA + NAD(P) = H+ + a uracil16 in tRNA + NAD(P)H.